glucagon processing [GO:0120116] (biological process) Definition: The formation of mature glucagon by proteolysis of the precursor proglucagon. References: PMID:28719828 Relationships: is a type of peptide hormone processing [GO:0016486]